{
  "gene": "UniProtKB:O95996",
  "gene_symbol": "APC2",
  "term_label": "negative regulation of canonical Wnt signaling pathway",
  "gene_name": "Adenomatous polyposis coli protein 2",
  "term_id": "GO:0090090"
}